{
  "gene": "UniProtKB:P78559",
  "term_id": "GO:0007409",
  "gene_symbol": "MAP1A",
  "gene_name": "Microtubule-associated protein 1A",
  "term_label": "axonogenesis"
}